{
  "term_id": "UNKNOWN:0001",
  "term_label": "Unknown molecular function",
  "gene_symbol": "ALPK3",
  "gene_name": "Alpha-protein kinase 3",
  "gene": "UniProtKB:Q96L96"
}